biofilm matrix assembly [GO:0098785] (biological process) Relationships: is a type of GO:0085029; is a type of biofilm matrix organization [GO:0098784]; is part of biofilm formation [GO:0042710] Definition: A process that results in the assembly of a biofilm matrix. Sources: GOC:mah